{
  "gene_symbol": "AKT3",
  "gene": "UniProtKB:Q9Y243",
  "gene_name": "RAC-gamma serine_threonine-protein kinase",
  "term_label": "protein serine/threonine kinase activity",
  "term_id": "GO:0004674"
}